{
  "term_id": "GO:0140374",
  "gene_symbol": "RIGI",
  "gene": "UniProtKB:O95786",
  "gene_name": "Antiviral innate immune response receptor RIG-I",
  "term_label": "antiviral innate immune response"
}